{
  "gene_symbol": "HLA-DQA2",
  "term_id": "GO:0050778",
  "term_label": "positive regulation of immune response",
  "gene": "UniProtKB:P01906",
  "gene_name": "HLA class II histocompatibility antigen, DQ alpha 2 chain"
}